{
  "gene": "UniProtKB:P08588",
  "term_id": "GO:0005886",
  "gene_symbol": "ADRB1",
  "gene_name": "Beta-1 adrenergic receptor",
  "term_label": "plasma membrane"
}